{
  "gene": "UniProtKB:P38936",
  "term_id": "GO:2000045",
  "gene_name": "Cyclin-dependent kinase inhibitor 1",
  "term_label": "regulation of G1/S transition of mitotic cell cycle",
  "gene_symbol": "CDKN1A"
}